{
  "term_id": "GO:0006412",
  "gene_symbol": "MRPL11",
  "term_label": "translation",
  "gene_name": "Large ribosomal subunit protein uL11m",
  "gene": "UniProtKB:Q9Y3B7"
}